N-terminal protein amino acid carbamoylation [GO:0050990] (biological process) Also known as: N-terminal protein amino acid carbamylation Relationships: is a type of N-terminal protein amino acid modification [GO:0031365] Definition: The carbamoylation of the N-terminal amino acid of proteins. Sources: GOC:ai